{
  "gene_name": "Ras association domain-containing protein 3",
  "term_label": "cytoplasm",
  "gene_symbol": "RASSF3",
  "gene": "UniProtKB:Q86WH2",
  "term_id": "GO:0005737"
}